{
  "gene_name": "Cysteine_serine-rich nuclear protein 3",
  "term_id": "GO:0043565",
  "gene": "UniProtKB:Q8WYN3",
  "gene_symbol": "CSRNP3",
  "term_label": "sequence-specific DNA binding"
}